{
  "term_id": "GO:0005789",
  "gene": "UniProtKB:Q9H819",
  "term_label": "endoplasmic reticulum membrane",
  "gene_symbol": "DNAJC18",
  "gene_name": "DnaJ homolog subfamily C member 18"
}